{
  "gene_symbol": "MED12",
  "term_label": "mediator complex",
  "term_id": "GO:0016592",
  "gene": "UniProtKB:Q93074",
  "gene_name": "Mediator of RNA polymerase II transcription subunit 12"
}